negative regulation of atrial cardiac muscle cell action potential [GO:1903948] (biological process) Relationships: is a type of GO:0045759; is a type of GO:0098910; is a type of negative regulation of cardiac muscle cell contraction [GO:0106135]; RO_0002212 atrial cardiac muscle cell action potential [GO:0086014] Definition: Any process that stops, prevents or reduces the frequency, rate or extent of atrial cardiac muscle cell action potential. Also known as: down regulation of atrial cardiac muscle cell action potential, down-regulation of atrial cardiac muscle cell action potential, downregulation of atrial cardiac muscle cell action potential, inhibition of atrial cardiac muscle cell action potential References: PMID:25281747 Sources: GOC:BHF, GOC:TermGenie, GOC:mtg_cardiac_conduct_nov11, GOC:nc, GO_REF:0000058